{
  "term_label": "ERAD pathway",
  "term_id": "GO:0036503",
  "gene": "UniProtKB:Q9UBS3",
  "gene_symbol": "DNAJB9",
  "gene_name": "DnaJ homolog subfamily B member 9"
}